{
  "gene": "UniProtKB:Q96MD2",
  "gene_name": "KICSTOR subunit 2",
  "gene_symbol": "KICS2",
  "term_id": "GO:0042149",
  "term_label": "cellular response to glucose starvation"
}